mitophagy [GO:0000423] (biological process) Subtypes: type 2 mitophagy [GO:0061734], type 1 mitophagy [GO:0180045] References: PMID:15798367 Relationships: is a type of autophagy of mitochondrion [GO:0000422]; is a type of GO:0016236 Note: Note that this terms refers to the macroautophagy process and is named by common usage. Be aware that there are a separate micromitophagy and mitophagy by induced vacuole formation processes. Regulation: regulated by regulation of mitophagy [GO:1901524]; negatively regulated by negative regulation of mitophagy [GO:1901525]; positively regulated by positive regulation of mitophagy [GO:1901526] Also known as: macromitophagy Definition: The selective autophagy process in which a mitochondrion is degraded by macroautophagy.